{
  "gene_symbol": "MT-CO1",
  "gene": "UniProtKB:P00395",
  "gene_name": "Cytochrome c oxidase subunit 1",
  "term_label": "aerobic respiration",
  "term_id": "GO:0009060"
}